{
  "gene": "UniProtKB:Q96RV3",
  "term_label": "Unknown molecular function",
  "gene_symbol": "PCNX1",
  "term_id": "UNKNOWN:0001",
  "gene_name": "Pecanex-like protein 1"
}